{
  "gene_symbol": "INSL6",
  "gene": "UniProtKB:Q9Y581",
  "gene_name": "Insulin-like peptide INSL6",
  "term_id": "UNKNOWN:0003",
  "term_label": "Unknown cellular component"
}